endoplasmic reticulum mannose trimming [GO:1904380] (BP) Also known as: ER mannose trimming, ER protein alpha-1,2-demannosylation, protein alpha-1,2-demannosylation in ER, protein alpha-1,2-demannosylation in ER quality control compartment, protein alpha-1,2-demannosylation in ERQC, protein alpha-1,2-demannosylation in endoplasmic reticulum, protein alpha-1,2-demannosylation in endoplasmic reticulum quality control compartment, glycoprotein mannose trimming in ER quality control compartment, glycoprotein mannose trimming in ER-derived quality control compartment, glycoprotein mannose trimming in ERQC, glycoprotein mannose trimming in endoplasmic reticulum quality control compartment, protein alpha-1,2-demannosylation in ER-derived quality control compartment References: PMID:24519966 Sources: GOC:PARL, GOC:TermGenie, GOC:bf, GO_REF:0000062 Subtypes: trimming of terminal mannose on C branch [GO:0036510] Definition: Any protein alpha-1,2-demannosylation that takes place in the endoplasmic reticulum quality control compartment (ERQC). Relationships: is a type of protein alpha-1,2-demannosylation [GO:0036508]; occurs in endoplasmic reticulum quality control compartment [GO:0044322]